{
  "gene": "UniProtKB:Q96DM1",
  "gene_symbol": "PGBD4",
  "term_label": "Unknown cellular component",
  "term_id": "UNKNOWN:0003",
  "gene_name": "PiggyBac transposable element-derived protein 4"
}